{
  "term_id": "GO:0030317",
  "gene_symbol": "CATSPER2",
  "gene": "UniProtKB:Q96P56",
  "term_label": "flagellated sperm motility",
  "gene_name": "Cation channel sperm-associated protein 2"
}